{
  "gene_symbol": "RAB40A",
  "term_id": "GO:0008021",
  "term_label": "synaptic vesicle",
  "gene_name": "Ras-related protein Rab-40A",
  "gene": "UniProtKB:Q8WXH6"
}